{
  "term_id": "GO:0000122",
  "term_label": "negative regulation of transcription by RNA polymerase II",
  "gene": "UniProtKB:Q96K62",
  "gene_symbol": "ZBTB45",
  "gene_name": "Zinc finger and BTB domain-containing protein 45"
}